centrosomal and pronuclear rotation [GO:0035047] (biological process) References: PMID:10085292 Sources: GOC:bf, ISBN:087969307X Definition: The rotation of centrosomes and associated pronuclei in one-cell embryos such as those of Caenorhabditis elegans, occurring as a transition between pronuclear migration and pronuclear fusion. Relationships: is a type of developmental process involved in reproduction [GO:0003006]; is a type of GO:0048869; BFO_0000050 GO:0007338